{
  "term_label": "cytoplasm",
  "gene": "UniProtKB:P06280",
  "gene_symbol": "GLA",
  "gene_name": "Alpha-galactosidase A",
  "term_id": "GO:0005737"
}